cyanophycin synthetase activity [GO:0043860] (molecular function) Subtypes: GO:0071160, cyanophycin synthetase activity (L-arginine-adding) [GO:0071161] Relationships: is a type of acid-amino acid ligase activity [GO:0016881] Also known as: cphA Definition: Catalysis of the ATP-dependent polymerization of arginine and aspartate to multi-L-arginyl-poly-L-aspartic acid (cyanophycin; a water-insoluble reserve polymer). Sources: GOC:jl